allene-oxide cyclase activity [GO:0046423] (molecular function) Also known as: (9Z)-(13S)-12,13-epoxyoctadeca-9,11,15-trienoate isomerase (cyclizing) Definition: Catalysis of the reaction: (9Z,13S,15Z)-12,13-epoxyoctadeca-9,11,15-trienoate = (15Z)-12-oxophyto-10,15-dienoate. Sources: EC:5.3.99.6, RHEA:22592 Relationships: is a type of cyclase activity [GO:0009975]; is a type of intramolecular oxidoreductase activity [GO:0016860]